{
  "term_id": "GO:0007099",
  "term_label": "centriole replication",
  "gene": "UniProtKB:Q8N137",
  "gene_name": "Centrobin",
  "gene_symbol": "CNTROB"
}